{
  "gene_symbol": "LEFTY1",
  "gene": "UniProtKB:O75610",
  "gene_name": "Left-right determination factor 1",
  "term_label": "anterior/posterior axis specification",
  "term_id": "GO:0009948"
}